{
  "gene_name": "Coiled-coil domain-containing protein 181",
  "term_id": "GO:0008017",
  "gene_symbol": "CCDC181",
  "gene": "UniProtKB:Q5TID7",
  "term_label": "microtubule binding"
}